{
  "gene": "UniProtKB:Q8NH92",
  "term_id": "GO:0005886",
  "gene_symbol": "OR1S1",
  "term_label": "plasma membrane",
  "gene_name": "Olfactory receptor 1S1"
}